Golgi membrane fusion [GO:0036504] (biological process) Definition: The joining of two lipid bilayers that surround the Golgi apparatus to form a single Golgi membrane. References: PMID:12473691 Sources: GOC:PARL, GOC:bf Also known as: Golgi apparatus membrane fusion, membrane fusion involved in Golgi reassembly, post-mitotic fusion of Golgi membranes Relationships: is a type of organelle membrane fusion [GO:0090174]; is part of GO:0090168